{
  "term_id": "UNKNOWN:0001",
  "term_label": "Unknown molecular function",
  "gene": "UniProtKB:Q3B820",
  "gene_symbol": "FAM161A",
  "gene_name": "Protein FAM161A"
}